{
  "term_id": "GO:0008266",
  "gene_name": "RNA-binding motif, single-stranded-interacting protein 3",
  "gene_symbol": "RBMS3",
  "term_label": "poly(U) RNA binding",
  "gene": "UniProtKB:Q6XE24"
}